{
  "term_id": "GO:0010880",
  "gene": "UniProtKB:P0DP23",
  "gene_name": "Calmodulin-1",
  "gene_symbol": "CALM1",
  "term_label": "regulation of release of sequestered calcium ion into cytosol by sarcoplasmic reticulum"
}